positive regulation of motor neuron axon guidance [GO:1905814] (biological process) Definition: Any process that activates or increases the frequency, rate or extent of motor neuron axon guidance. References: PMID:18434533 Sources: GOC:TermGenie, GO_REF:0000058 Also known as: positive regulation of motoneuron axon guidance, positive regulation of motor axon guidance, positive regulation of motor axon pathfinding, up regulation of motoneuron axon guidance, up regulation of motor axon guidance, up regulation of motor axon pathfinding, up regulation of motor neuron axon guidance, up-regulation of motoneuron axon guidance, up-regulation of motor axon guidance, up-regulation of motor axon pathfinding, up-regulation of motor neuron axon guidance, upregulation of motoneuron axon guidance, upregulation of motor axon guidance, upregulation of motor axon pathfinding, upregulation of motor neuron axon guidance, activation of motoneuron axon guidance, activation of motor axon guidance, activation of motor axon pathfinding, activation of motor neuron axon guidance Relationships: is_a GO:1902669; is a type of regulation of motor neuron axon guidance [GO:1905812]; RO_0002213 motor neuron axon guidance [GO:0008045]